regulation of non-professional antigen presenting cell antigen processing and presentation [GO:0002619] (biological process) Relationships: is a type of regulation of antigen processing and presentation [GO:0002577]; regulates non-professional antigen presenting cell antigen processing and presentation [GO:0002473] Subtypes: negative regulation of non-professional antigen presenting cell antigen processing and presentation [GO:0002620], positive regulation of non-professional antigen presenting cell antigen processing and presentation [GO:0002621] Definition: Any process that modulates the frequency, rate, or extent of non-professional antigen presenting cell antigen processing and presentation. Sources: GOC:add